{
  "gene_symbol": "LGSN",
  "term_id": "GO:0016020",
  "term_label": "membrane",
  "gene_name": "Lengsin",
  "gene": "UniProtKB:Q5TDP6"
}